urethanase activity [GO:0050387] (molecular function) Definition: Catalysis of the reaction: H2O + H+ + urethane = CO2 + ethanol + NH4. Relationships: is a type of GO:0016811 Sources: EC:3.5.1.75, RHEA:21372 Also known as: urethane amidohydrolase (decarboxylating), urethane hydrolase activity